{
  "gene_name": "Protein BNIP5",
  "term_id": "UNKNOWN:0002",
  "gene": "UniProtKB:P0C671",
  "term_label": "Unknown biological process",
  "gene_symbol": "BNIP5"
}